W chromosome [GO:0000804] (cellular component) Relationships: is a type of sex chromosome [GO:0000803] References: PMID:20622855 Sources: GOC:mah, GOC:mr, ISBN:0321000382 Definition: The sex chromosome present in females of species in which the female is the heterogametic sex; generally, the sex chromosome that pairs with the Z chromosome in the heterogametic sex. The W chromosome is absent from the cells of males and present in one copy in the somatic cells of females.